DNA replication, Okazaki fragment processing [GO:0033567] (biological process) Sources: GOC:mah, ISBN:0716720094 Subtypes: GO:1903461 Definition: The DNA metabolic process, occurring during lagging strand synthesis, by which RNA primers are removed from Okazaki fragments, the resulting gaps filled by DNA polymerization, and the ends ligated to form a continuous strand. Relationships: is a type of GO:0006259; is part of lagging strand elongation [GO:0006273]